{
  "gene_name": "Leucine-rich repeat and guanylate kinase domain-containing protein",
  "term_id": "UNKNOWN:0002",
  "term_label": "Unknown biological process",
  "gene": "UniProtKB:Q96M69",
  "gene_symbol": "LRGUK"
}